leukotriene-E4 20-monooxygenase activity [GO:0050052] (molecular function) Also known as: leukotriene-E4 w-hydroxylase activity, (7E,9E,11Z,14Z)-(5S,6R)-6-(cystein-S-yl)-5-hydroxyicosa-7,9,11,14-tetraenoate,NADPH:oxygen oxidoreductase (20-hydroxylating), leukotriene-E(4) omega-hydroxylase activity, leukotriene-E4 omega-hydroxylase activity Sources: EC:1.14.13.34, RHEA:24120 Relationships: is a type of oxidoreductase activity, acting on paired donors, with incorporation or reduction of molecular oxygen, NAD(P)H as one donor, and incorporation of one atom of oxygen [GO:0016709] Definition: Catalysis of the reaction: H+ + leukotriene E(4) + NADPH + O2 = 20-hydroxy-leukotriene E(4) + H2O + NADP+.